{
  "term_label": "myo-inositol transport",
  "gene": "UniProtKB:Q96QE2",
  "gene_name": "Proton myo-inositol cotransporter",
  "term_id": "GO:0015798",
  "gene_symbol": "SLC2A13"
}